nucleoside diphosphate catabolic process [GO:0009134] (BP) Relationships: is a type of nucleoside diphosphate metabolic process [GO:0009132]; is a type of nucleoside phosphate catabolic process [GO:1901292] Also known as: nucleoside diphosphate breakdown, nucleoside diphosphate catabolism, nucleoside diphosphate degradation Definition: The chemical reactions and pathways resulting in the breakdown of a nucleoside diphosphate, a compound consisting of a nucleobase linked to a deoxyribose or ribose sugar esterified with diphosphate on the sugar. Subtypes: purine nucleoside diphosphate catabolic process [GO:0009137], pyrimidine nucleoside diphosphate catabolic process [GO:0009140], GO:0009191, deoxyribonucleoside diphosphate catabolic process [GO:0009192] Sources: GOC:go_curators, ISBN:0198506732